{
  "gene_name": "E3 SUMO-protein ligase PIAS4",
  "term_label": "transcription coregulator activity",
  "gene": "UniProtKB:Q8N2W9",
  "gene_symbol": "PIAS4",
  "term_id": "GO:0003712"
}